{
  "gene_name": "Paraneoplastic antigen Ma6E",
  "term_id": "UNKNOWN:0001",
  "gene_symbol": "PNMA6E",
  "term_label": "Unknown molecular function",
  "gene": "UniProtKB:A0A0J9YXQ4"
}